{
  "term_label": "serine-type endopeptidase inhibitor activity",
  "gene": "UniProtKB:P36952",
  "gene_name": "Serpin B5",
  "gene_symbol": "SERPINB5",
  "term_id": "GO:0004867"
}